{
  "gene": "UniProtKB:O14796",
  "term_label": "Unknown biological process",
  "gene_symbol": "SH2D1B",
  "gene_name": "SH2 domain-containing protein 1B",
  "term_id": "UNKNOWN:0002"
}